stomatal complex morphogenesis [GO:0010103] (biological process) Relationships: is a type of plant epidermis morphogenesis [GO:0090626]; is a type of post-embryonic plant morphogenesis [GO:0090698]; is part of shoot system morphogenesis [GO:0010016]; is part of stomatal complex development [GO:0010374] Definition: The process in which the anatomical structures of the stomatal complex are generated and organized. The stomatal complex is the stomatal guard cells and their associated epidermal cells. Sources: GOC:tair_curators